{
  "term_id": "GO:0043235",
  "gene_name": "Tyrosine-protein kinase receptor UFO",
  "gene": "UniProtKB:P30530",
  "term_label": "receptor complex",
  "gene_symbol": "AXL"
}